{
  "gene_symbol": "GHRH",
  "gene_name": "Somatoliberin",
  "term_label": "perikaryon",
  "term_id": "GO:0043204",
  "gene": "UniProtKB:P01286"
}